mediator complex assembly [GO:0036034] (biological process) Relationships: is a type of protein-containing complex assembly [GO:0065003] Regulation: regulated by regulation of mediator complex assembly [GO:2001176]; negatively regulated by negative regulation of mediator complex assembly [GO:2001177]; positively regulated by positive regulation of mediator complex assembly [GO:2001178] Definition: The aggregation, arrangement and bonding together of a set of components to form a mediator complex. The mediator complex is a protein complex that interacts with the carboxy-terminal domain of the largest subunit of RNA polymerase II and plays an active role in transducing the signal from a transcription factor to the transcriptional machinery. The Saccharomyces complex contains several identifiable subcomplexes: a head domain comprising Srb2, -4, and -5, Med6, -8, and -11, and Rox3 proteins; a middle domain comprising Med1, -4, and -7, Nut1 and -2, Cse2, Rgr1, Soh1, and Srb7 proteins; a tail consisting of Gal11p, Med2p, Pgd1p, and Sin4p; and a regulatory subcomplex comprising Ssn2, -3, and -8, and Srb8 proteins. Metazoan mediator complexes have similar modular structures and include homologs of yeast Srb and Med proteins. References: PMID:17641689 Sources: GOC:yaf